{
  "gene_name": "SCP2 sterol-binding domain-containing protein 1",
  "gene_symbol": "SCP2D1",
  "gene": "UniProtKB:Q9UJQ7",
  "term_label": "cytosol",
  "term_id": "GO:0005829"
}